preribosome, small subunit precursor [GO:0030688] (cellular component) Relationships: is a type of preribosome [GO:0030684] Note: Note that this complex is 43S in Saccharomyces. References: PMID:10567516 Also known as: 43S preribosome Definition: A preribosomal complex consisting of 20S pre-rRNA, ribosomal proteins including late-associating small subunit proteins, and associated proteins; a precursor of the eukaryotic cytoplasmic small ribosomal subunit.